{
  "term_label": "Unknown cellular component",
  "gene_symbol": "DEFB104A",
  "term_id": "UNKNOWN:0003",
  "gene": "UniProtKB:Q8WTQ1",
  "gene_name": "Beta-defensin 104"
}